{
  "gene": "UniProtKB:Q9BTC0",
  "term_id": "UNKNOWN:0001",
  "gene_symbol": "DIDO1",
  "gene_name": "Death-inducer obliterator 1",
  "term_label": "Unknown molecular function"
}